{
  "term_label": "positive regulation of DNA-templated transcription",
  "gene": "UniProtKB:Q9UMN6",
  "term_id": "GO:0045893",
  "gene_symbol": "KMT2B",
  "gene_name": "Histone-lysine N-methyltransferase 2B"
}